{
  "gene": "UniProtKB:P18848",
  "term_id": "GO:1990589",
  "gene_symbol": "ATF4",
  "term_label": "ATF4-CREB1 transcription factor complex",
  "gene_name": "Cyclic AMP-dependent transcription factor ATF-4"
}